heparan sulfate proteoglycan binding [GO:0043395] (MF) Also known as: heparin proteoglycan binding Definition: Binding to a heparan sulfate proteoglycan, any proteoglycan containing heparan sulfate as the glycosaminoglycan carbohydrate unit. Relationships: is_a proteoglycan binding [GO:0043394] Sources: ISBN:0198506732